plasma membrane protein complex [GO:0098797] (cellular component) Relationships: is a type of membrane protein complex [GO:0098796]; is part of plasma membrane [GO:0005886] Definition: Any protein complex that is part of the plasma membrane. Subtypes: plasma membrane proton-transporting V-type ATPase, V0 domain [GO:0000222], plasma membrane proton-transporting V-type ATPase, V1 domain [GO:0000223], voltage-gated sodium channel complex [GO:0001518], caveolar macromolecular signaling complex [GO:0002095], membrane attack complex [GO:0005579], heterotrimeric G-protein complex [GO:0005834], GO:0005889, GO:0005890, GO:0005891, GO:0005922, voltage-gated potassium channel complex [GO:0008076], GO:0008282, D-amino-acid dehydrogenase complex [GO:0009324], auxin efflux carrier complex [GO:0009921], dystrophin-associated glycoprotein complex [GO:0016010], GO:0016011, GO:0016012, syntrophin complex [GO:0016013], GO:0016014, inaD signaling complex [GO:0016027], catenin complex [GO:0016342], GO:0016600, GO:0016935, histamine-gated chloride channel complex [GO:0019183], plasma membrane-derived photosystem I [GO:0030094], plasma membrane-derived thylakoid photosystem II [GO:0030096], AP-2 adaptor complex [GO:0030122], GO:0030132, GO:0030936, death-inducing signaling complex [GO:0031264], contractile vacuole pore [GO:0031913], GO:0032997, plasma membrane proton-transporting V-type ATPase complex [GO:0033181], TAT protein transport complex [GO:0033281], GO:0033573, CFTR-NHERF-ezrin complex [GO:0034662], GO:0034673, SC5b-7 complex [GO:0034995], alphav-beta5 integrin-vitronectin complex [GO:0034997], subapical complex [GO:0035003], alphav-beta3 integrin-PKCalpha complex [GO:0035866], alphav-beta3 integrin-IGF-1-IGF1R complex [GO:0035867], GO:0035868, MHC protein complex [GO:0042611], NADPH oxidase complex [GO:0043020], ATP-binding cassette (ABC) transporter complex [GO:0043190], GO:0044731, GO:0044799, plasma membrane-derived thylakoid ribulose bisphosphate carboxylase complex [GO:0048493], GO:0062136, GO:0070014, alphav-beta3 integrin-thrombospondin complex [GO:0070017], interleukin-12-interleukin-12 receptor complex [GO:0070023], CD19-Vav-PIK3R1 complex [GO:0070024], alphav-beta3 integrin-osteopontin complex [GO:0070029], alphav-beta1 integrin-osteopontin complex [GO:0070030], alphav-beta5 integrin-osteopontin complex [GO:0070031], alpha6-beta4 integrin-Shc-Grb2 complex [GO:0070333], alpha6-beta4 integrin-laminin 5 complex [GO:0070334], alphav-beta3 integrin-CD47 complex [GO:0070357], Shc-EGFR complex [GO:0070435], Grb2-EGFR complex [GO:0070436], GO:0070437, interleukin4-interleukin-4 receptor complex [GO:0070450], alphav-beta3 integrin-collagen alpha3(VI) complex [GO:0070464], alpha1-beta1 integrin-alpha3(VI) complex [GO:0070465], GO:0070466, alphaIIb-beta3 integrin-talin complex [GO:0070515], GO:0070518, alpha4-beta1 integrin-CD63 complex [GO:0070519], alpha4-beta1 integrin-CD81 complex [GO:0070520], alpha4-beta1 integrin-CD82 complex [GO:0070521], alphaM-beta2 integrin-CD63 complex [GO:0070558], Grb2-Sos complex [GO:0070618], Shc-Grb2-Sos complex [GO:0070619], EGFR-Grb2-Sos complex [GO:0070620], EGFR-Shc-Grb2-Sos complex [GO:0070621], GO:0070718, GO:0070719, Grb2-SHP-2 complex [GO:0070720], Delta1 complex [GO:0070763], gamma-secretase-Delta1 complex [GO:0070764], GO:0070765, GO:0070769, alphaIIb-beta3 integrin-CD47-FAK complex [GO:0070770], alphaIIb-beta3 integrin-CD47-Src complex [GO:0070771], alpha9-beta1 integrin-ADAM1 complex [GO:0071052], alpha9-beta1 integrin-ADAM2 complex [GO:0071053], alpha9-beta1 integrin-ADAM3 complex [GO:0071054], GO:0071055, alpha9-beta1 integrin-ADAM15 complex [GO:0071056], GO:0071057, alpha3-beta1 integrin-CD151 complex [GO:0071058], GO:0071059, alpha7-beta1 integrin-CD151 complex [GO:0071060], GO:0071061, GO:0071062, GO:0071064, alpha9-beta1 integrin-vascular cell adhesion molecule-1 complex [GO:0071065], alphav-beta3 integrin-ADAM23 complex [GO:0071067], alpha9-beta1 integrin-ADAM12 complex [GO:0071068], alpha4-beta1 integrin-thrombospondin-1 complex [GO:0071069], alpha4-beta1 integrin-thrombospondin-2 complex [GO:0071070], fibronectin-tissue transglutaminase complex [GO:0071078], alpha2-beta1 integrin-chondroadherin complex [GO:0071079], alpha3-beta1 integrin-basigin complex [GO:0071080], alpha3-beta1 integrin-CD63 complex [GO:0071081], alpha9-beta1 integrin-tenascin complex [GO:0071082], alphaV-beta3 integrin-CD47-FCER2 complex [GO:0071083], alpha2-beta1 integrin-CD47 complex [GO:0071084], alphaIIb-beta3 integrin-CD9 complex [GO:0071085], alphaIIb-beta3 integrin-CD9-CD47-platelet glycoprotein Ib complex [GO:0071086], alpha11-beta1 integrin-collagen type I complex [GO:0071087], alpha5-beta1 integrin-tissue transglutaminase complex [GO:0071088], alphaV-beta3 integrin-tissue transglutaminase complex [GO:0071089], alphaIIb-beta3 integrin-fibronectin-tissue transglutaminase complex [GO:0071090], alpha1-beta1 integrin-tissue transglutaminase complex [GO:0071091], alpha3-beta1 integrin-tissue transglutaminase complex [GO:0071092], alpha5-beta1 integrin-fibronectin-tissue transglutaminase complex [GO:0071093], alpha6-beta4 integrin-CD9 complex [GO:0071094], alpha3-beta1 integrin-thrombospondin complex [GO:0071095], alphaV-beta3 integrin-gelsolin complex [GO:0071096], alphaV-beta3 integrin-paxillin-Pyk2 complex [GO:0071097], alpha6-beta4 integrin-Fyn complex [GO:0071098], GO:0071099, alphaV-beta8 integrin-MMP14-TGFbeta-1 complex [GO:0071100], alpha4-beta1 integrin-JAM2 complex [GO:0071101], alpha4-beta1 integrin-paxillin complex [GO:0071102], alpha4-beta4 integrin-EMILIN-1 complex [GO:0071112], alphaIIb-beta3 integrin-ICAM-4 complex [GO:0071113], alphaV-beta3 integrin-tumstatin complex [GO:0071114], alpha5-beta1 integrin-endostatin complex [GO:0071115], GO:0071116, GO:0071117, alphaV-beta3 integrin-NOV complex [GO:0071118], GO:0071119, alpha4-beta1 integrin-CD47 complex [GO:0071120], alpha9-beta1 integrin-VEGF-D complex [GO:0071121], alpha9-beta1 integrin-VEGF-A complex [GO:0071122], GO:0071123, alpha1-beta1 integrin-tyrosine-protein phosphatase non-receptor type 2 complex [GO:0071124], alphaV-beta3 integrin-EGFR complex [GO:0071125], GO:0071126, alpha9-beta1 integrin-osteopontin complex [GO:0071127], alpha5-beta1 integrin-osteopontin complex [GO:0071128], GO:0071129, alpha5-beta1 integrin-LPP3 complex [GO:0071130], alphaV-beta3 integrin-laminin alpha-4 complex [GO:0071131], alphaX-beta2 integrin-ICAM-4 complex [GO:0071132], alpha9-beta1 integrin-ADAM8 complex [GO:0071133], alpha9-beta1 integrin-thrombospondin-1 complex [GO:0071134], GO:0071135, GO:0071136, alphaV-beta3 integrin-CD98 complex [GO:0071137], GO:0071138, GO:0071183, MPP7-DLG1-LIN7 complex [GO:0097025], ciliary necklace [GO:0097538], plasma membrane signaling receptor complex [GO:0098802], bacterial-type flagellum stator complex [GO:0120101], MalFGK2 complex [GO:1990176], amino acid transport complex [GO:1990184], GO:1990203, GO:1990207, platelet-derived growth factor receptor-ligand complex [GO:1990270], EFF-1 complex [GO:1990392], GO:1990398, GO:1990851 Sources: GOC:dos